L-tyrosine biosynthetic process from chorismate via 4-hydroxyphenylpyruvate [GO:0019292] (biological process) Definition: The chemical reactions and pathways resulting in the formation of L-tyrosine from other compounds, including chorismate, via the intermediate 4-hydroxyphenylpyruvate. Sources: GOC:go_curators Also known as: tyrosine biosynthetic process from chorismate via 4-hydroxyphenylpyruvate, L-tyrosine anabolism from chorismate via 4-hydroxyphenylpyruvate, L-tyrosine biosynthetic process from chorismate via p-hydroxyphenylpyruvate, L-tyrosine formation from chorismate via 4-hydroxyphenylpyruvate, L-tyrosine synthesis from chorismate via 4-hydroxyphenylpyruvate Relationships: is a type of L-tyrosine biosynthetic process [GO:0006571]; is_a chorismate metabolic process [GO:0046417]